{
  "gene_name": "ETS translocation variant 2",
  "term_label": "regulation of transcription by RNA polymerase II",
  "gene": "UniProtKB:O00321",
  "term_id": "GO:0006357",
  "gene_symbol": "ETV2"
}